{
  "gene_symbol": "SLC12A7",
  "term_id": "GO:0055064",
  "term_label": "chloride ion homeostasis",
  "gene": "UniProtKB:Q9Y666",
  "gene_name": "Solute carrier family 12 member 7"
}